{
  "term_label": "purine nucleoside transmembrane transport",
  "term_id": "GO:0015860",
  "gene_name": "Solute carrier family 28 member 3",
  "gene": "UniProtKB:Q9HAS3",
  "gene_symbol": "SLC28A3"
}